{
  "term_label": "spermatid development",
  "gene_name": "Androglobin",
  "gene": "UniProtKB:Q8N7X0",
  "gene_symbol": "ADGB",
  "term_id": "GO:0007286"
}